ligase activity, forming nitrogen-metal bonds [GO:0051002] (molecular function) Relationships: is a type of ligase activity [GO:0016874] Subtypes: ligase activity, forming nitrogen-metal bonds, forming coordination complexes [GO:0051003] Sources: EC:6.6.-.- Definition: Catalysis of the joining of a metal ion to a molecule via a nitrogen-metal bond, with the concomitant hydrolysis of the diphosphate bond in ATP or a similar triphosphate.